averantin hydroxylase activity [GO:0140395] (molecular function) References: PMID:8368836 Sources: EC:1.14.14.116 Relationships: is a type of oxidoreductase activity, acting on paired donors, with incorporation or reduction of molecular oxygen [GO:0016705]; is part of aflatoxin biosynthetic process [GO:0045122] Definition: Catalyzes the reaction: (1'S)-averantin + [reduced NADPH--hemoprotein reductase] + O2 = (1'S,5'S)-5'-hydroxyaverantin + [oxidized NADPH--hemoprotein reductase] + H2O. Involved in aflatoxin biosynthesis.